{
  "gene_symbol": "LOC124905412",
  "gene": "UniProtKB:A0A1B0GW55",
  "term_id": "GO:0005634",
  "gene_name": "Homeobox domain-containing protein",
  "term_label": "nucleus"
}